{
  "gene_symbol": "SLC25A26",
  "term_id": "GO:0005743",
  "term_label": "mitochondrial inner membrane",
  "gene": "UniProtKB:Q70HW3",
  "gene_name": "Mitochondrial S-adenosylmethionine carrier protein"
}